endonucleolytic cleavage of tetracistronic rRNA transcript (SSU-rRNA, 5.8S rRNA, 2S rRNA, LSU-rRNA) [GO:0000483] (biological process) Definition: Endonucleolytic cleavage of a pre-rRNA molecule originally produced as a tetracistronic rRNA transcript that contains the Small SubUnit (SSU) rRNA, the 5.8S rRNA, 2S rRNA, and the Large SubUnit (LSU) rRNA, in that order, from 5' to 3' along the primary transcript. Primary ribosomal RNA transcripts with four genes, in this order, are produced in the nuclei of D. melanogaster as well as in those of other dipteran species. Relationships: is a type of rRNA processing [GO:0006364] Subtypes: cleavage between SSU-rRNA and 5.8S rRNA of tetracistronic rRNA transcript (SSU-rRNA, 5.8S rRNA, 2S rRNA, LSU-rRNA) [GO:0000484], cleavage between 2S rRNA and LSU-rRNA of tetracistronic rRNA transcript (SSU-rRNA, 5.8S rRNA, 2S rRNA, LSU-rRNA) [GO:0000485], GO:0000486 Sources: GOC:curators